{
  "gene": "UniProtKB:Q6ZWJ1",
  "gene_name": "Syntaxin-binding protein 4",
  "term_label": "cytoplasmic vesicle",
  "term_id": "GO:0031410",
  "gene_symbol": "STXBP4"
}